{
  "term_id": "GO:0006015",
  "gene_symbol": "PRPS1L1",
  "gene": "UniProtKB:P21108",
  "term_label": "5-phosphoribose 1-diphosphate biosynthetic process",
  "gene_name": "Ribose-phosphate pyrophosphokinase 3"
}